{
  "term_label": "calcium-dependent phospholipid binding",
  "gene": "UniProtKB:P27216",
  "gene_symbol": "ANXA13",
  "gene_name": "Annexin A13",
  "term_id": "GO:0005544"
}